cholesterol 7-desaturase [NAD(P)H] activity [GO:0170056] (molecular function) Definition: Catalysis of the reaction: cholesterol + H+ + NAD(P)H + O2 = 7-dehydrocholesterol + 2 H2O + NAD(P)+. Also known as: C-7 cholesterol dehydrogenase, cholesterol 7,8-dehydrogenase References: PMID:21632547, PMID:31521708 Sources: EC:1.14.19.21 Relationships: is a type of sterol desaturase activity [GO:0070704]